{
  "gene": "UniProtKB:Q16851",
  "term_label": "UTP:glucose-1-phosphate uridylyltransferase activity",
  "gene_name": "UTP--glucose-1-phosphate uridylyltransferase",
  "gene_symbol": "UGP2",
  "term_id": "GO:0003983"
}